{
  "term_label": "regulation of transcription by RNA polymerase II",
  "gene_symbol": "CSRNP1",
  "term_id": "GO:0006357",
  "gene": "UniProtKB:Q96S65",
  "gene_name": "Cysteine_serine-rich nuclear protein 1"
}